regulation of NMDA receptor activity [GO:2000310] (biological process) Also known as: regulation of N-methyl-D-aspartate selective glutamate receptor activity Sources: GOC:BHF Subtypes: negative regulation of NMDA glutamate receptor activity [GO:1904782] Relationships: is a type of regulation of transmembrane transporter activity [GO:0022898]; is a type of regulation of neurotransmitter receptor activity [GO:0099601]; regulates NMDA glutamate receptor activity [GO:0004972] Definition: Any process that modulates the frequency, rate or extent of N-methyl-D-aspartate selective glutamate receptor activity.